{
  "term_label": "interleukin-10-mediated signaling pathway",
  "gene_symbol": "LILRA2",
  "gene": "UniProtKB:Q8N149",
  "term_id": "GO:0140105",
  "gene_name": "Leukocyte immunoglobulin-like receptor subfamily A member 2"
}